D-xylose 1-dehydrogenase (NAD+) activity [GO:0047838] (molecular function) Sources: RHEA:13861 Definition: Catalysis of the reaction: D-xylose + NAD+ = D-xylonolactone + NADH. Also known as: D-xylose 1-dehydrogenase (NAD) activity, (NAD)-linked D-xylose dehydrogenase activity, D-xylose dehydrogenase activity, D-xylose:NAD+ 1-oxidoreductase activity, NAD-D-xylose, NAD-D-xylose dehydrogenase activity, NAD-linked D-xylose dehydrogenase activity Relationships: is a type of GO:0016616